{
  "gene_symbol": "SUN3",
  "gene_name": "SUN domain-containing protein 3",
  "term_id": "GO:0005635",
  "term_label": "nuclear envelope",
  "gene": "UniProtKB:Q8TAQ9"
}